angioblast cell migration [GO:0035476] (BP) Definition: The orderly movement of angioblasts, cells involved in blood vessel morphogenesis. Relationships: is_a cell migration [GO:0016477]; is part of blood vessel morphogenesis [GO:0048514] Subtypes: angioblast cell migration involved in selective angioblast sprouting [GO:0035475], angioblast cell migration from lateral mesoderm to midline [GO:0035479] References: PMID:19815777 Sources: GOC:dgh